{
  "gene_name": "cGMP-gated cation channel alpha-1",
  "gene": "UniProtKB:P29973",
  "term_id": "GO:0005223",
  "gene_symbol": "CNGA1",
  "term_label": "intracellularly cGMP-activated cation channel activity"
}